hydroxyversicolorone reductase activity [GO:0102974] (molecular function) Sources: RHEA:35691 Relationships: is a type of oxidoreductase activity, acting on the CH-OH group of donors, NAD or NADP as acceptor [GO:0016616] Definition: Catalysis of the reaction: versicolorone + NADP = hydroxyversicolorone + NADPH.